{
  "gene_name": "Calcium_calmodulin-dependent protein kinase type 1B",
  "term_label": "calmodulin binding",
  "gene": "UniProtKB:Q6P2M8",
  "gene_symbol": "PNCK",
  "term_id": "GO:0005516"
}